{
  "term_id": "GO:0005634",
  "term_label": "nucleus",
  "gene_name": "Serine_threonine-protein kinase VRK1",
  "gene_symbol": "VRK1",
  "gene": "UniProtKB:Q99986"
}